{
  "term_label": "Unknown molecular function",
  "gene_name": "Anaphase-promoting complex subunit 4",
  "gene": "UniProtKB:Q9UJX5",
  "gene_symbol": "ANAPC4",
  "term_id": "UNKNOWN:0001"
}